vesicle uncoating [GO:0072319] (biological process) Sources: GOC:mah Also known as: vesicle coat disassembly Subtypes: Golgi vesicle uncoating [GO:0048212], clathrin coat disassembly [GO:0072318], COPII vesicle uncoating [GO:0090112] Relationships: is a type of protein depolymerization [GO:0051261]; BFO_0000050 GO:0016192 Definition: A protein depolymerization process that results in the disassembly of vesicle coat proteins.